{
  "term_id": "GO:0009755",
  "gene_name": "Steroidogenic factor 1",
  "gene": "UniProtKB:Q13285",
  "term_label": "hormone-mediated signaling pathway",
  "gene_symbol": "NR5A1"
}